{
  "gene_name": "snRNA-activating protein complex subunit 1",
  "term_id": "GO:0042795",
  "gene_symbol": "SNAPC1",
  "gene": "UniProtKB:Q16533",
  "term_label": "snRNA transcription by RNA polymerase II"
}